{
  "term_label": "'de novo' NAD+ biosynthetic process from L-tryptophan",
  "gene": "UniProtKB:P14902",
  "gene_name": "Indoleamine 2,3-dioxygenase 1",
  "term_id": "GO:0034354",
  "gene_symbol": "IDO1"
}